{
  "gene_symbol": "PSG3",
  "gene": "UniProtKB:Q16557",
  "gene_name": "Pregnancy-specific beta-1-glycoprotein 3",
  "term_id": "UNKNOWN:0002",
  "term_label": "Unknown biological process"
}